{
  "gene": "UniProtKB:Q9BUZ4",
  "gene_symbol": "TRAF4",
  "gene_name": "TNF receptor-associated factor 4",
  "term_id": "GO:0035591",
  "term_label": "signaling adaptor activity"
}